Bcl-2 family protein complex [GO:0097136] (cellular component) Subtypes: BAD-BCL-xl complex [GO:0097137], BAD-BCL-2 complex [GO:0097138], BID-BCL-2 complex [GO:0097139], BIM-BCL-xl complex [GO:0097140], BIM-BCL-2 complex [GO:0097141], GO:0097142, GO:0097143, GO:0097144, GO:0097145, NOXA-BCL-xl complex [GO:0097146], NOXA-BCL-2 complex [GO:0097147], BCL-2 complex [GO:0097148] References: PMID:14634621 Sources: GOC:so Relationships: is a type of GO:0032991 Definition: A protein complex that consists of members of the Bcl-2 family of anti- and proapoptotic regulators. Bcl-2 proteins respond to cues from various forms of intracellular stress, such as DNA damage or cytokine deprivation, and interact with opposing family members to determine whether or not the caspase proteolytic cascade should be unleashed.